{
  "gene": "UniProtKB:O14683",
  "term_label": "Unknown cellular component",
  "gene_name": "Tumor protein p53-inducible protein 11",
  "gene_symbol": "TP53I11",
  "term_id": "UNKNOWN:0003"
}